translocation of peptides or proteins into host [GO:0042000] (biological process) Definition: The directed movement of peptides or proteins produced by an organism to a location inside its host organism. The host is defined as the larger of the organisms involved in a symbiotic interaction. References: PMID:15953025, PMID:18406478 Sources: GOC:cc Also known as: translocation of peptides or proteins into other organism during symbiotic interaction, translocation of peptides or proteins into other organism involved in symbiotic interaction, transport of peptides or proteins into other organism during symbiotic interaction, transport of peptides or proteins into host Relationships: is a type of translocation of molecules into host [GO:0044417] Subtypes: translocation of peptides or proteins into host cell cytoplasm [GO:0044053]